{
  "term_id": "GO:0000151",
  "gene_symbol": "RNF144B",
  "term_label": "ubiquitin ligase complex",
  "gene": "UniProtKB:Q7Z419",
  "gene_name": "E3 ubiquitin-protein ligase RNF144B"
}